{
  "term_id": "GO:0005634",
  "term_label": "nucleus",
  "gene_name": "MOB kinase activator 3C",
  "gene": "UniProtKB:Q70IA8",
  "gene_symbol": "MOB3C"
}